{
  "gene_symbol": "LDAH",
  "term_id": "GO:0004771",
  "term_label": "sterol ester esterase activity",
  "gene": "UniProtKB:Q9H6V9",
  "gene_name": "Lipid droplet-associated hydrolase"
}